{
  "term_label": "molecular adaptor activity",
  "term_id": "GO:0060090",
  "gene_symbol": "SEPTIN1",
  "gene": "UniProtKB:Q8WYJ6",
  "gene_name": "Septin-1"
}